{
  "gene_name": "Cadherin-like protein 26",
  "term_label": "adherens junction organization",
  "gene": "UniProtKB:Q8IXH8",
  "term_id": "GO:0034332",
  "gene_symbol": "CDH26"
}